{
  "gene": "UniProtKB:A0A075B6S0",
  "gene_symbol": "TRGJ1",
  "term_label": "Unknown biological process",
  "gene_name": "T cell receptor gamma joining 1",
  "term_id": "UNKNOWN:0002"
}